{
  "term_label": "trans-Golgi network",
  "term_id": "GO:0005802",
  "gene_symbol": "ATP8B1",
  "gene_name": "Phospholipid-transporting ATPase IC",
  "gene": "UniProtKB:O43520"
}